{
  "gene_symbol": "IL1RAPL2",
  "term_id": "GO:0005886",
  "gene": "UniProtKB:Q9NP60",
  "gene_name": "X-linked interleukin-1 receptor accessory protein-like 2",
  "term_label": "plasma membrane"
}